fungal-type cell wall disassembly [GO:0071853] (biological process) Subtypes: GO:1904541 Relationships: is a type of GO:0031505; is a type of cell wall disassembly [GO:0044277] Definition: A cellular process that results in the breakdown of a fungal-type cell wall. Sources: GOC:mah